{
  "term_id": "GO:1901741",
  "gene_symbol": "SCGB3A1",
  "gene_name": "Secretoglobin family 3A member 1",
  "gene": "UniProtKB:Q96QR1",
  "term_label": "positive regulation of myoblast fusion"
}